lateral cortical node [GO:1990463] (cellular component) References: PMID:25009287 Sources: GOC:mah Relationships: is a type of protein-containing complex [GO:0032991]; is part of lateral cell cortex [GO:0097575] Definition: A protein complex that is anchored at the cortical face of the plasma membrane, and contains proteins involved in regulating cell cycle progression. In Schizosaccharomyces pombe, lateral cortical nodes are several megadaltons in size, and contain Slf1, which anchors the complex at the membrane, and the methyltransferase Skb1 in stoichiometric quantities, and may contain other proteins. Also known as: Skb1-containing cortical node